{
  "term_id": "UNKNOWN:0003",
  "gene_name": "Organic anion transporter 3",
  "term_label": "Unknown cellular component",
  "gene": "UniProtKB:Q8TCC7",
  "gene_symbol": "SLC22A8"
}